{
  "gene_name": "Dendritic cell nuclear protein 1",
  "gene_symbol": "DCANP1",
  "gene": "UniProtKB:Q8TF63",
  "term_label": "nucleoplasm",
  "term_id": "GO:0005654"
}